{
  "term_id": "UNKNOWN:0002",
  "gene_symbol": "KIAA1191",
  "gene": "UniProtKB:Q96A73",
  "term_label": "Unknown biological process",
  "gene_name": "Putative monooxygenase p33MONOX"
}